{
  "term_id": "UNKNOWN:0001",
  "gene": "UniProtKB:O60637",
  "gene_symbol": "TSPAN3",
  "term_label": "Unknown molecular function",
  "gene_name": "Tetraspanin-3"
}